glial cytoplasmic inclusion [GO:0097409] (cellular component) Definition: Non-membrane-bound cytoplasmic inclusions composed of 10-40 nm granule-coated fibrils. These inclusions have an abnormal accumulation of alpha-synuclein protein and are found in association with multiple system atrophy. References: PMID:21562886, PMID:2559165 Sources: NIF_Subcellular:nlx_subcell_20090703 Also known as: GCI, Papp-Lantos body Relationships: is a type of inclusion body [GO:0016234]